{
  "gene": "UniProtKB:Q8NEZ3",
  "term_label": "intraciliary transport particle A",
  "term_id": "GO:0030991",
  "gene_symbol": "WDR19",
  "gene_name": "WD repeat-containing protein 19"
}